inductive mesenchymal-endodermal cell signaling [GO:0060494] (BP) Subtypes: mesenchymal-endodermal cell signaling involved in lung induction [GO:0060493] Sources: GOC:dph, GOC:mtg_lung Also known as: inductive mesenchymal-endodermal cell signalling Relationships: is a type of GO:0031129 Definition: Any process that mediates the transfer of information from a mesenchymal cell to an endodermal cell changing the fate of the endodermal cell.